{
  "gene": "UniProtKB:O75920",
  "gene_symbol": "SERF1B",
  "gene_name": "Small EDRK-rich factor 1",
  "term_id": "UNKNOWN:0001",
  "term_label": "Unknown molecular function"
}